ureide catabolic process [GO:0010136] (biological process) Relationships: is a type of catabolic process [GO:0009056]; is a type of amide metabolic process [GO:0043603] Definition: The chemical reactions and pathways resulting in the breakdown of ureide, which is the organic form of nitrogen in nitrogen fixing and transporting plants with the release of ammonium. Also known as: ureide breakdown, ureide catabolism, ureide degradation Sources: GOC:pz